{
  "term_label": "retinol metabolic process",
  "gene_name": "Retinol dehydrogenase 8",
  "gene": "UniProtKB:Q9NYR8",
  "gene_symbol": "RDH8",
  "term_id": "GO:0042572"
}